membrane lipid catabolic process [GO:0046466] (biological process) Sources: GOC:ai Also known as: membrane lipid peroxidation, membrane lipid breakdown, membrane lipid catabolism, membrane lipid degradation Subtypes: glycolipid catabolic process [GO:0019377], GO:0030149 Definition: The chemical reactions and pathways resulting in the breakdown of membrane lipids, any lipid found in or associated with a biological membrane. Relationships: is a type of GO:0006643; is a type of lipid catabolic process [GO:0016042]